negative regulation of viral life cycle [GO:1903901] (biological process) Also known as: down regulation of viral life cycle, down-regulation of viral life cycle, downregulation of viral life cycle, down regulation of viral assembly, maturation, egress, and release, down-regulation of viral assembly, maturation, egress, and release, downregulation of viral assembly, maturation, egress, and release, inhibition of viral assembly, maturation, egress, and release, inhibition of viral life cycle, negative regulation of viral assembly, maturation, egress, and release, down regulation of lytic viral life cycle, down regulation of viral infectious cycle, down regulation of viral replication, down-regulation of lytic viral life cycle, down-regulation of viral infectious cycle, down-regulation of viral replication, downregulation of lytic viral life cycle, downregulation of viral infectious cycle, downregulation of viral replication, inhibition of lytic viral life cycle, inhibition of viral infectious cycle, inhibition of viral replication, negative regulation of lytic viral life cycle, negative regulation of viral infectious cycle, negative regulation of viral replication References: PMID:18005716 Sources: GOC:TermGenie, GO_REF:0000058 Definition: Any process that stops, prevents or reduces the frequency, rate or extent of viral life cycle. Subtypes: GO:1901253, negative regulation of viral budding via host ESCRT complex [GO:1903773] Relationships: is a type of negative regulation of viral process [GO:0048525]; is a type of regulation of viral life cycle [GO:1903900]; negatively regulates GO:0019058